{
  "gene_name": "RCC1-like G exchanging factor-like protein",
  "term_id": "GO:0008053",
  "gene_symbol": "RCC1L",
  "term_label": "mitochondrial fusion",
  "gene": "UniProtKB:Q96I51"
}